{
  "gene_name": "Chromatin assembly factor 1 subunit A",
  "term_label": "nucleosome assembly",
  "gene": "UniProtKB:Q13111",
  "term_id": "GO:0006334",
  "gene_symbol": "CHAF1A"
}